{
  "term_id": "GO:0012505",
  "gene_symbol": "STX1A",
  "gene_name": "Syntaxin-1A",
  "term_label": "endomembrane system",
  "gene": "UniProtKB:Q16623"
}